{
  "term_label": "regulation of apoptotic process",
  "gene_name": "Ubiquitin carboxyl-terminal hydrolase 17-like protein 17",
  "term_id": "GO:0042981",
  "gene": "UniProtKB:D6RBQ6",
  "gene_symbol": "USP17L17"
}